{
  "term_label": "insulin receptor signaling pathway",
  "term_id": "GO:0008286",
  "gene_symbol": "APPL1",
  "gene_name": "DCC-interacting protein 13-alpha",
  "gene": "UniProtKB:Q9UKG1"
}